{
  "gene_symbol": "PLCH1",
  "term_id": "GO:0005737",
  "gene": "UniProtKB:Q4KWH8",
  "gene_name": "1-phosphatidylinositol 4,5-bisphosphate phosphodiesterase eta-1",
  "term_label": "cytoplasm"
}